{
  "gene_symbol": "SCP2D1-AS1",
  "term_label": "Unknown biological process",
  "gene": "UniProtKB:Q9BR46",
  "term_id": "UNKNOWN:0002",
  "gene_name": "Putative uncharacterized protein SCP2D1-AS1"
}